{
  "gene": "UniProtKB:Q9UPE1",
  "term_label": "nucleus",
  "gene_symbol": "SRPK3",
  "term_id": "GO:0005634",
  "gene_name": "SRSF protein kinase 3"
}